climbing fiber [GO:0044301] (cellular component) Sources: NIF_Subcellular:nlx_subcell_20090203 Also known as: climbing fibre Definition: The axon of inferior olive neuron that projects to the cerebellar cortex, largely via the inferior cerebellar peduncle. They range in diameter from 1-3 um and are myelinated until they enter the granule cell layer. They give off collaterals to the deep cerebellar nuclei. They synapse extensively with the dendrites of Purkinje cells in the molecular layer, where each fiber branches repeatedly to climb along the Purkinje cell dendritic tree. Each Purkinje cell is innervated by only a single climbing fiber. Relationships: is a type of GO:0030424